tRNA-specific adenosine deaminase activity [GO:0008251] (molecular function) Subtypes: GO:0043829, GO:0052717 Sources: GOC:mah Relationships: is a type of adenosine deaminase activity [GO:0004000]; is a type of GO:0140101 Definition: Catalysis of the reaction: adenosine + H2O = inosine + NH3, in a tRNA molecule. Also known as: tRNA-adenosine deaminase activity